{
  "gene": "UniProtKB:Q9BYD3",
  "term_id": "UNKNOWN:0002",
  "term_label": "Unknown biological process",
  "gene_name": "Large ribosomal subunit protein uL4m",
  "gene_symbol": "MRPL4"
}